{
  "term_id": "UNKNOWN:0002",
  "gene": "UniProtKB:Q5JY77",
  "gene_symbol": "GPRASP1",
  "term_label": "Unknown biological process",
  "gene_name": "G-protein coupled receptor-associated sorting protein 1"
}